{
  "term_id": "GO:0030674",
  "term_label": "protein-macromolecule adaptor activity",
  "gene_symbol": "GOLGA5",
  "gene": "UniProtKB:Q8TBA6",
  "gene_name": "Golgin subfamily A member 5"
}